{
  "gene": "UniProtKB:Q92598",
  "gene_symbol": "HSPH1",
  "term_id": "GO:0005634",
  "gene_name": "Heat shock protein 105 kDa",
  "term_label": "nucleus"
}